viral genome maturation [GO:0019070] (biological process) References: PMID:21490093 Sources: GOC:pk Relationships: is a type of viral process [GO:0016032]; is part of virion assembly [GO:0019068] Definition: The processes involved in creating a mature, stable viral genome. Begins after genome replication with a newly synthesized nucleic acid and ends when the genome is ready to be packaged. Includes the addition of proteins to the newly synthesized genome, and DNA repair processes.